{
  "gene_name": "Bromodomain-containing protein 7",
  "gene": "UniProtKB:Q9NPI1",
  "term_label": "nucleus",
  "term_id": "GO:0005634",
  "gene_symbol": "BRD7"
}